{
  "gene_name": "Putative inactive group IIC secretory phospholipase A2",
  "gene_symbol": "PLA2G2C",
  "gene": "UniProtKB:Q5R387",
  "term_label": "Unknown cellular component",
  "term_id": "UNKNOWN:0003"
}